{
  "gene_name": "Sphingosine 1-phosphate receptor 4",
  "term_id": "GO:0007189",
  "gene": "UniProtKB:O95977",
  "gene_symbol": "S1PR4",
  "term_label": "adenylate cyclase-activating G protein-coupled receptor signaling pathway"
}